{
  "gene": "UniProtKB:Q9H6I2",
  "term_id": "GO:0007507",
  "term_label": "heart development",
  "gene_name": "Transcription factor SOX-17",
  "gene_symbol": "SOX17"
}